interleukin-7 production [GO:0032636] (biological process) Definition: The appearance of interleukin-7 due to biosynthesis or secretion following a cellular stimulus, resulting in an increase in its intracellular or extracellular levels. Also known as: IL-7 production, interleukin-7 biosynthetic process, interleukin-7 secretion Regulation: regulated by GO:0032676; negatively regulated by negative regulation of interleukin-7 production [GO:0032716]; positively regulated by GO:0032756 Sources: GOC:mah Relationships: is a type of cytokine production [GO:0001816]